cell septum edging catabolic process [GO:0030995] (BP) Also known as: septum edging hydrolysis, cell septum edging hydrolysis, hydrolysis of cell septum edging, hydrolysis of edging of cell septum References: PMID:15194814 Sources: GOC:mah Relationships: is a type of GO:0000272; is part of septum digestion after cytokinesis [GO:0000920] Definition: The chemical reactions and pathways resulting in the dissolution of the septum edging during cell separation.